{
  "gene_symbol": "CD22",
  "gene": "UniProtKB:P20273",
  "term_id": "GO:0042609",
  "gene_name": "B-cell receptor CD22",
  "term_label": "CD4 receptor binding"
}